{
  "gene_symbol": "TRIM49",
  "gene": "UniProtKB:P0CI25",
  "term_id": "GO:0045087",
  "term_label": "innate immune response",
  "gene_name": "Tripartite motif-containing protein 49"
}